acetylpyruvate hydrolase activity [GO:0018773] (molecular function) Also known as: 2,4-dioxopentanoate acetylhydrolase activity Relationships: is a type of GO:0016823 Sources: RHEA:16097 Definition: Catalysis of the reaction: acetylpyruvate + H2O = acetate + H+ + pyruvate.